reorganization of host cellular membranes to establish sites of replication [GO:0140755] (biological process) Relationships: is a type of viral process [GO:0016032]; is_a symbiont-mediated perturbation of host membrane [GO:0141171] References: PMID:34699787, PMID:4372566 Definition: A process in which a virus triggers host intracellular membranes to be reorganized, forming membranous webs, which are thought to be the site of replication or certain viruses, for example the HPV virus.